negative regulation of protein K48-linked deubiquitination [GO:1903094] (BP) Relationships: is a type of negative regulation of protein deubiquitination [GO:0090086]; is a type of regulation of protein K48-linked deubiquitination [GO:1903093]; negatively regulates GO:0071108 References: PMID:21097510 Sources: GOC:PARL, GOC:TermGenie, GOC:bf, GO_REF:0000058 Also known as: down regulation of protein K48-linked deubiquitination, down-regulation of protein K48-linked deubiquitination, downregulation of protein K48-linked deubiquitination, inhibition of protein K48-linked deubiquitination Definition: Any process that stops, prevents or reduces the frequency, rate or extent of protein K48-linked deubiquitination.